{
  "gene": "UniProtKB:P36896",
  "term_label": "cellular response to growth factor stimulus",
  "gene_name": "Activin receptor type-1B",
  "term_id": "GO:0071363",
  "gene_symbol": "ACVR1B"
}